{
  "term_label": "cytosol",
  "gene_symbol": "CFTR",
  "term_id": "GO:0005829",
  "gene": "UniProtKB:P13569",
  "gene_name": "Cystic fibrosis transmembrane conductance regulator"
}